{
  "term_label": "Golgi membrane",
  "term_id": "GO:0000139",
  "gene_name": "Protein SYS1 homolog",
  "gene": "UniProtKB:Q8N2H4",
  "gene_symbol": "SYS1"
}